{
  "term_id": "UNKNOWN:0002",
  "gene_symbol": "LRRC31",
  "term_label": "Unknown biological process",
  "gene_name": "Leucine-rich repeat-containing protein 31",
  "gene": "UniProtKB:Q6UY01"
}